{
  "gene": "UniProtKB:P23409",
  "gene_name": "Myogenic factor 6",
  "gene_symbol": "MYF6",
  "term_id": "UNKNOWN:0003",
  "term_label": "Unknown cellular component"
}